{
  "gene_name": "Type I iodothyronine deiodinase",
  "gene": "UniProtKB:P49895",
  "term_label": "Unknown cellular component",
  "gene_symbol": "DIO1",
  "term_id": "UNKNOWN:0003"
}